Schwann cell microvillus [GO:0097454] (cellular component) Definition: Small finger-like extension of a Schwann cell that contacts the nodal membrane. References: PMID:15988042 Sources: NIF_Subcellular:sao1890444066 Relationships: is a type of microvillus [GO:0005902]; is_a glial cell projection [GO:0097386]